{
  "gene_symbol": "ABCG5",
  "gene_name": "ATP-binding cassette sub-family G member 5",
  "term_id": "GO:0033344",
  "gene": "UniProtKB:Q9H222",
  "term_label": "cholesterol efflux"
}